{
  "gene_name": "Sorbin and SH3 domain-containing protein 1",
  "gene": "UniProtKB:Q9BX66",
  "term_label": "cell-substrate junction",
  "term_id": "GO:0030055",
  "gene_symbol": "SORBS1"
}